negative regulation of arginine catabolic process [GO:1900082] (biological process) Also known as: down regulation of arginine breakdown, down regulation of arginine catabolic process, down regulation of arginine catabolism, down regulation of arginine degradation, down-regulation of arginine breakdown, down-regulation of arginine catabolic process, down-regulation of arginine catabolism, down-regulation of arginine degradation, downregulation of arginine breakdown, downregulation of arginine catabolic process, downregulation of arginine catabolism, downregulation of arginine degradation, negative regulation of arginine breakdown, negative regulation of arginine catabolism, negative regulation of arginine degradation, inhibition of arginine breakdown, inhibition of arginine catabolic process, inhibition of arginine catabolism, inhibition of arginine degradation Definition: Any process that stops, prevents or reduces the frequency, rate or extent of arginine catabolic process. Sources: GOC:TermGenie, GOC:dgf Relationships: is a type of GO:0033242; is a type of negative regulation of amino acid metabolic process [GO:0045763]; is a type of negative regulation of small molecule metabolic process [GO:0062014]; is a type of regulation of arginine catabolic process [GO:1900081]; negatively regulates GO:0006527